regulation of muscle hypertrophy [GO:0014743] (biological process) Relationships: is a type of regulation of muscle system process [GO:0090257]; regulates muscle hypertrophy [GO:0014896] Definition: Any process that modulates the frequency, rate or extent of muscle hypertrophy. Sources: GOC:mtg_muscle Subtypes: regulation of cardiac muscle hypertrophy [GO:0010611], GO:0014741, positive regulation of muscle hypertrophy [GO:0014742], regulation of myofibril size [GO:0014881], regulation of skeletal muscle hypertrophy [GO:1904204], GO:1905147